cytoplasmic U snRNP body [GO:0071254] (cellular component) Relationships: is a type of cytoplasmic ribonucleoprotein granule [GO:0036464] References: PMID:17595295 Sources: GOC:sart Also known as: U body, U-body Definition: A focus in the cytoplasm that contains uridine-rich small nuclear ribonucleoproteins (U snRNPs) and essential snRNP assembly factors. These U bodies are invariably found in association with P bodies.